peptide cross-linking via L-cystine [GO:0018316] (BP) Sources: RESID:AA0025 Relationships: is a type of peptide cross-linking [GO:0018149]; is a type of peptidyl-cysteine modification [GO:0018198] Definition: The oxidation of two peptidyl-cysteine residues to form a peptidyl-L-cystine (dicysteine) in which segments of peptide chain are linked by a disulfide bond; the cross-link may be between different or the same peptide chain.